{
  "gene_name": "Small ribosomal subunit protein uS2B",
  "term_label": "ribosomal small subunit assembly",
  "gene_symbol": "RPSA2",
  "gene": "UniProtKB:A0A8I5KQE6",
  "term_id": "GO:0000028"
}